{
  "gene_name": "1-phosphatidylinositol 4,5-bisphosphate phosphodiesterase beta-3",
  "term_label": "cytoplasm",
  "term_id": "GO:0005737",
  "gene_symbol": "PLCB3",
  "gene": "UniProtKB:Q01970"
}